{
  "gene_symbol": "H6PD",
  "gene_name": "GDH_6PGL endoplasmic bifunctional protein",
  "term_label": "endoplasmic reticulum",
  "term_id": "GO:0005783",
  "gene": "UniProtKB:O95479"
}